symbiont-mediated disruption of host cell envelope [GO:0098933] (biological process) Definition: The process in which a symbiont effects a change that impairs the structure or function of the host cell envelope. The host is defined as the larger of the organisms involved in a symbiotic interaction. Sources: ISBN:0198547684 Also known as: disruption by symbiont of host cell envelope Relationships: is a type of symbiont-mediated disruption of host cellular anatomical structure [GO:0052008] Subtypes: symbiont-mediated disruption of host cell wall [GO:0052009], symbiont entry into host cell via disruption of host cell envelope [GO:0098994], symbiont entry into host cell via disruption of host cell glycocalyx [GO:0098996]